{
  "gene_symbol": "RBFA",
  "gene": "UniProtKB:Q8N0V3",
  "term_label": "Unknown cellular component",
  "term_id": "UNKNOWN:0003",
  "gene_name": "Putative ribosome-binding factor A, mitochondrial"
}